{
  "term_id": "GO:0035005",
  "gene_symbol": "PIK3CA",
  "gene_name": "Phosphatidylinositol 4,5-bisphosphate 3-kinase catalytic subunit alpha isoform",
  "term_label": "1-phosphatidylinositol-4-phosphate 3-kinase activity",
  "gene": "UniProtKB:P42336"
}